{
  "term_id": "GO:0005737",
  "term_label": "cytoplasm",
  "gene_name": "Neuronatin",
  "gene": "UniProtKB:Q16517",
  "gene_symbol": "NNAT"
}